{
  "gene_symbol": "CCR5",
  "gene": "UniProtKB:P51681",
  "term_id": "GO:0009897",
  "gene_name": "C-C chemokine receptor type 5",
  "term_label": "external side of plasma membrane"
}